nephrocyte diaphragm [GO:0005917] (cellular component) References: PMID:18971929 Sources: GOC:mtg_kidney_jan10, GOC:sart Also known as: nephrocyte junction Definition: A specialized cell-cell junction found between nephrocytes of the insect kidney, which is adapted for filtration of hemolymph. The insect nephrocyte is anatomically and functionally similar to the glomerular podocyte of vertebrates. Relationships: is a type of filtration diaphragm [GO:0036056]